{
  "term_label": "neuron projection",
  "gene": "UniProtKB:Q9P2E2",
  "gene_symbol": "KIF17",
  "gene_name": "Kinesin-like protein KIF17",
  "term_id": "GO:0043005"
}